{
  "term_label": "Unknown biological process",
  "gene_symbol": "SAMD9L",
  "gene_name": "Sterile alpha motif domain-containing protein 9-like",
  "gene": "UniProtKB:Q8IVG5",
  "term_id": "UNKNOWN:0002"
}